{
  "term_id": "GO:0031398",
  "term_label": "positive regulation of protein ubiquitination",
  "gene_symbol": "BIRC3",
  "gene_name": "Baculoviral IAP repeat-containing protein 3",
  "gene": "UniProtKB:Q13489"
}